{
  "term_id": "UNKNOWN:0002",
  "gene_symbol": "RBBP8NL",
  "gene": "UniProtKB:Q8NC74",
  "gene_name": "RBBP8 N-terminal-like protein",
  "term_label": "Unknown biological process"
}